positive regulation of leukocyte apoptotic process [GO:2000108] (biological process) Subtypes: positive regulation of mast cell apoptotic process [GO:0033027], positive regulation of neutrophil apoptotic process [GO:0033031], positive regulation of lymphocyte apoptotic process [GO:0070230], positive regulation of macrophage apoptotic process [GO:2000111], positive regulation of dendritic cell apoptotic process [GO:2000670] Relationships: is_a GO:0043065; is a type of regulation of leukocyte apoptotic process [GO:2000106]; positively regulates GO:0071887 Definition: Any process that activates or increases the frequency, rate or extent of leukocyte apoptotic process. Sources: GOC:BHF, GOC:mtg_apoptosis Also known as: positive regulation of leukocyte apoptosis